{
  "gene_symbol": "FBXO47",
  "gene_name": "F-box only protein 47",
  "term_label": "Unknown biological process",
  "term_id": "UNKNOWN:0002",
  "gene": "UniProtKB:Q5MNV8"
}